{
  "term_id": "GO:0007274",
  "term_label": "neuromuscular synaptic transmission",
  "gene_name": "Neuronal acetylcholine receptor subunit alpha-6",
  "gene_symbol": "CHRNA6",
  "gene": "UniProtKB:Q15825"
}